alpha-pinene metabolic process [GO:0018867] (BP) Definition: The chemical reactions and pathways involving alpha-pinene, a monoterpene that may be a significant factor affecting bacterial activities in nature. It is a major component in tea-tree oils, and gives off a piney smelling odor. Relationships: is a type of pinene metabolic process [GO:0033073] Also known as: alpha-pinene metabolism Subtypes: GO:0046248, GO:0046249 Sources: UM-BBD_pathwayID:apn